{
  "term_label": "adenylate cyclase-activating G protein-coupled receptor signaling pathway",
  "gene_symbol": "LPAR3",
  "gene": "UniProtKB:Q9UBY5",
  "gene_name": "Lysophosphatidic acid receptor 3",
  "term_id": "GO:0007189"
}